{
  "term_label": "detection of chemical stimulus involved in sensory perception of bitter taste",
  "gene_symbol": "TAS2R13",
  "gene": "UniProtKB:Q9NYV9",
  "term_id": "GO:0001580",
  "gene_name": "Taste receptor type 2 member 13"
}